{
  "term_id": "UNKNOWN:0003",
  "term_label": "Unknown cellular component",
  "gene": "UniProtKB:Q8TB69",
  "gene_name": "Zinc finger protein 519",
  "gene_symbol": "ZNF519"
}